{
  "gene_symbol": "ATF6",
  "gene": "UniProtKB:P18850",
  "term_label": "nucleus",
  "term_id": "GO:0005634",
  "gene_name": "Cyclic AMP-dependent transcription factor ATF-6 alpha"
}